DNA template activity [GO:0000497] (molecular function) Definition: Binding to nucleic acid via hydrogen bonds between the bases of a gene product molecule and the bases of a target DNA molecule. Sources: GOC:krc Also known as: base pairing with DNA Note: Note that with respect to annotation, "base pairing" and its child terms are intended to be used to annotate the activity of gene products composed of nucleic acid, presumably RNA, to interact with DNA molecules via base pairing. Internal base pairing with itself is considered part of the secondary structure of the molecule and is not within the scope of GO function. Relationships: is_a DNA binding [GO:0003677]; is a type of molecular template activity [GO:0140489] Subtypes: template for synthesis of G-rich strand of telomere DNA activity [GO:0000332]